{
  "term_id": "GO:0007605",
  "gene_symbol": "COL11A2",
  "term_label": "sensory perception of sound",
  "gene": "UniProtKB:P13942",
  "gene_name": "Collagen alpha-2(XI) chain"
}